{
  "gene_symbol": "RHCG",
  "term_label": "basolateral plasma membrane",
  "term_id": "GO:0016323",
  "gene": "UniProtKB:Q9UBD6",
  "gene_name": "Ammonium transporter Rh type C"
}